{
  "term_id": "GO:0005344",
  "gene": "UniProtKB:P02144",
  "gene_symbol": "MB",
  "term_label": "oxygen carrier activity",
  "gene_name": "Myoglobin"
}